{
  "term_label": "Unknown molecular function",
  "gene": "UniProtKB:O95297",
  "term_id": "UNKNOWN:0001",
  "gene_symbol": "MPZL1",
  "gene_name": "Myelin protein zero-like protein 1"
}